{
  "gene": "UniProtKB:Q8NEV8",
  "gene_symbol": "EXPH5",
  "term_label": "endosome",
  "gene_name": "Exophilin-5",
  "term_id": "GO:0005768"
}